{
  "gene_symbol": "JPH2",
  "term_id": "GO:0016529",
  "gene": "UniProtKB:Q9BR39",
  "term_label": "sarcoplasmic reticulum",
  "gene_name": "Junctophilin-2"
}